{
  "term_id": "UNKNOWN:0001",
  "gene": "UniProtKB:Q2KHR3",
  "gene_symbol": "QSER1",
  "term_label": "Unknown molecular function",
  "gene_name": "Glutamine and serine-rich protein 1"
}